deoxyribonuclease inhibitor activity [GO:0060703] (molecular function) Sources: GOC:dph, GOC:tb Also known as: DNase inhibitor activity Definition: Binds to and stops, prevents or reduces the activity of deoxyribonuclease. Relationships: is a type of nuclease inhibitor activity [GO:0140721]; negatively regulates DNA nuclease activity [GO:0004536]